succinyl-CoA binding [GO:0120226] (molecular function) Relationships: is a type of acyl-CoA binding [GO:0120227] Definition: Binding to succinyl-CoA, an omega-carboxyacyl-CoA having succinoyl as the S-acyl component. Also known as: succinyl-coenzyme A binding Sources: GOC:krc